{
  "gene": "UniProtKB:P09105",
  "gene_name": "Hemoglobin subunit theta-1",
  "term_label": "erythrocyte development",
  "gene_symbol": "HBQ1",
  "term_id": "GO:0048821"
}